inner ear receptor cell stereocilium organization [GO:0060122] (biological process) Subtypes: auditory receptor cell stereocilium organization [GO:0060088], vestibular receptor cell stereocilium organization [GO:0060121], GO:0120045 Sources: GOC:dph Also known as: inner ear hair cell receptor stereocilium organization, inner ear receptor stereocilium organisation, inner ear receptor stereocilium organization and biogenesis Relationships: is a type of neuron projection development [GO:0031175]; is part of inner ear receptor cell development [GO:0060119] Definition: A process that is carried out at the cellular level which results in the assembly, arrangement of constituent parts, or disassembly of a stereocilium. A stereocilium is an actin-based protrusion from the apical surface of inner ear receptor cells.